negative regulation of starch biosynthetic process [GO:7770012] (biological process) Relationships: is a type of negative regulation of macromolecule biosynthetic process [GO:0010558]; is a type of regulation of starch biosynthetic process [GO:0010581]; is a type of negative regulation of carbohydrate metabolic process [GO:0045912]; negatively regulates starch biosynthetic process [GO:0019252] Definition: Any process that stops, prevents, or reduces the frequency, rate or extent of the chemical reactions and pathways resulting in the formation of starch. References: PMID:26554020